{
  "gene_name": "U4_U6.U5 small nuclear ribonucleoprotein 27 kDa protein",
  "term_id": "UNKNOWN:0001",
  "term_label": "Unknown molecular function",
  "gene": "UniProtKB:Q8WVK2",
  "gene_symbol": "SNRNP27"
}